{
  "gene": "UniProtKB:A0A8V8TPW1",
  "term_id": "UNKNOWN:0001",
  "gene_name": "Uncharacterized protein",
  "term_label": "Unknown molecular function",
  "gene_symbol": "A0A8V8TPW1"
}